{
  "gene_name": "Kunitz-type protease inhibitor 3",
  "term_id": "UNKNOWN:0003",
  "term_label": "Unknown cellular component",
  "gene_symbol": "SPINT3",
  "gene": "UniProtKB:P49223"
}